{
  "term_label": "endoplasmic reticulum",
  "gene_name": "Lysophosphatidylcholine acyltransferase 2",
  "term_id": "GO:0005783",
  "gene_symbol": "LPCAT2",
  "gene": "UniProtKB:Q7L5N7"
}